{
  "gene": "UniProtKB:Q96QZ0",
  "gene_name": "Pannexin-3",
  "term_label": "plasma membrane",
  "gene_symbol": "PANX3",
  "term_id": "GO:0005886"
}